ferrous iron binding [GO:0008198] (MF) Relationships: is a type of iron ion binding [GO:0005506] Definition: Binding to a ferrous iron ion, Fe(II). Sources: GOC:ai